polyol transmembrane transport [GO:0015791] (biological process) Relationships: is a type of organic hydroxy compound transport [GO:0015850]; is a type of transmembrane transport [GO:0055085] Definition: The directed movement of polyols, any polyhydric alcohol, across a membrane. Sources: GOC:ai Subtypes: arabinitol transmembrane transport [GO:0015792], glycerol transmembrane transport [GO:0015793], GO:0015795, GO:0015796, GO:0015797, chloramphenicol transmembrane transport [GO:0042892], glucosylglycerol transmembrane transport [GO:0051475], GO:1902341, myo-inositol import across plasma membrane [GO:1904679], autoinducer AI-2 transmembrane transport [GO:1905887]